{
  "term_label": "Unknown molecular function",
  "term_id": "UNKNOWN:0001",
  "gene_name": "PR domain zinc finger protein 13",
  "gene": "UniProtKB:Q9H4Q3",
  "gene_symbol": "PRDM13"
}